{
  "gene_name": "Glycerol-3-phosphate acyltransferase 1, mitochondrial",
  "gene": "UniProtKB:Q9HCL2",
  "term_id": "GO:0006650",
  "term_label": "glycerophospholipid metabolic process",
  "gene_symbol": "GPAM"
}